{
  "term_label": "succinate-CoA ligase complex (ADP-forming)",
  "gene_symbol": "SUCLG1",
  "gene_name": "Succinate--CoA ligase [ADP_GDP-forming] subunit alpha, mitochondrial",
  "gene": "UniProtKB:P53597",
  "term_id": "GO:0009361"
}